protein polymerization [GO:0051258] (biological process) Definition: The process of creating protein polymers, compounds composed of a large number of component monomers; polymeric proteins may be made up of different or identical monomers. Polymerization occurs by the addition of extra monomers to an existing poly- or oligomeric protein. Regulation: regulated by regulation of protein polymerization [GO:0032271]; negatively regulated by negative regulation of protein polymerization [GO:0032272]; RO_0002213 by positive regulation of protein polymerization [GO:0032273] Subtypes: free ubiquitin chain polymerization [GO:0010994], actin filament polymerization [GO:0030041], intermediate filament polymerization [GO:0045107], microtubule polymerization [GO:0046785] Sources: GOC:ai Also known as: protein polymer biosynthesis, protein polymer biosynthetic process, protein polymer formation Relationships: is a type of protein-containing complex assembly [GO:0065003]